{
  "gene": "UniProtKB:P06748",
  "term_label": "ribosomal large subunit export from nucleus",
  "term_id": "GO:0000055",
  "gene_name": "Nucleophosmin",
  "gene_symbol": "NPM1"
}